cytosolic proteasome core complex [GO:0031603] (cellular component) Definition: The core complex of a proteasome located in the cytosol of a cell. Sources: GOC:mah, GOC:mtg_sensu Relationships: is a type of proteasome core complex [GO:0005839]; is part of cytosolic proteasome complex [GO:0031597]